{
  "gene": "UniProtKB:Q9BZJ8",
  "term_label": "plasma membrane",
  "gene_name": "G-protein coupled receptor 61",
  "gene_symbol": "GPR61",
  "term_id": "GO:0005886"
}